{
  "term_id": "UNKNOWN:0002",
  "term_label": "Unknown biological process",
  "gene_symbol": "SUV39H1",
  "gene": "UniProtKB:O43463",
  "gene_name": "Histone-lysine N-methyltransferase SUV39H1"
}